{
  "gene_symbol": "BCAN",
  "term_label": "synapse",
  "term_id": "GO:0045202",
  "gene_name": "Brevican core protein",
  "gene": "UniProtKB:Q96GW7"
}